{
  "term_label": "Unknown molecular function",
  "gene_symbol": "TACC2",
  "term_id": "UNKNOWN:0001",
  "gene": "UniProtKB:O95359",
  "gene_name": "Transforming acidic coiled-coil-containing protein 2"
}